orexigenic neuropeptide QRFP receptor binding [GO:0031854] (molecular function) Definition: Binding to an orexigenic neuropeptide QRFP receptor. Sources: GOC:mah, GOC:nln Also known as: orexigenic neuropeptide QRFP receptor ligand Relationships: is a type of neuropeptide receptor binding [GO:0071855]